{
  "gene_symbol": "IL18R1",
  "gene": "UniProtKB:Q13478",
  "term_label": "interleukin-18 receptor activity",
  "gene_name": "Interleukin-18 receptor 1",
  "term_id": "GO:0042008"
}